{
  "gene": "UniProtKB:P29074",
  "term_label": "protein tyrosine phosphatase activity",
  "gene_name": "Tyrosine-protein phosphatase non-receptor type 4",
  "gene_symbol": "PTPN4",
  "term_id": "GO:0004725"
}